inactivation of paternal X chromosome by genomic imprinting [GO:0060818] (biological process) Definition: Compensating for the two-fold variation in X-chromosome:autosome ratios between sexes by a global inactivation of all, or most of, the genes on the paternal X-chromosome in the XX sex by genomic imprinting. References: PMID:11743158, PMID:16789828, PMID:18425126, PMID:23578369 Sources: GOC:dph, GOC:sdb_2009, GOC:tb Also known as: iXCI, inactivation of paternal X chromosome by genetic imprinting Note: Imprinting controlled inactivation of the paternal X chromosome appears to be the ancestral form of sex chromosome inactivation in therian mammals. In eutherian mammals, imprinted X inactivation (iXCI) has largely been replaced by random X inactivation in a process regulated by the Xist and additional ncRNA's encoded within the "choice" region of the X chromosome. In a few mammals with early zygotic genome activation, imprinted X inactivation of the paternal X chromsome occurs very early during embryonic development. Imprinted iXCI has been observed in mice, rats, and bovines, and is best studied in mice where it occurs in the 4 cell stage in mice. In epiblast cells which will become the embryo proper, the inactivated paternal X chromosome is reactivated and dosage compensation of the X chromosome is regenerated by random X inactivation in embryonic tissues. In extraembryonic tissues, the selective inactivation of the paternal chromosome remains and is essential for proper development of the placenta. Selective inactivation of the paternal X chromosome via imprinting is the only form of X chromosome inactivation in marsupials, though the mechanism there may be significantly different in marsupials as the Xist transcript is not present on metatherian X chromosomes. Relationships: is a type of dosage compensation by inactivation of X chromosome [GO:0009048]; is a type of GO:0071514